regulation of mRNA stability involved in cellular response to UV [GO:1902629] (biological process) Also known as: regulation of mRNA stability involved in cellular response to UV light stimulus, regulation of mRNA stability involved in cellular response to UV radiation stimulus, regulation of mRNA stability involved in cellular response to ultraviolet light stimulus, regulation of mRNA stability involved in cellular response to ultraviolet radiation stimulus Relationships: is a type of regulation of mRNA stability [GO:0043488]; is part of cellular response to UV [GO:0034644] References: PMID:10954610 Sources: GOC:TermGenie, GO_REF:0000060 Definition: Any regulation of mRNA stability that is involved in cellular response to UV.